regulation of tonic skeletal muscle contraction [GO:0014746] (biological process) Subtypes: positive regulation of tonic skeletal muscle contraction [GO:0014747], GO:0014748 Sources: GOC:mtg_muscle Definition: Any process that modulates the frequency, rate or extent of tonic skeletal muscle contraction. Relationships: is a type of GO:0014819; regulates tonic skeletal muscle contraction [GO:0014720]